{
  "gene": "UniProtKB:P00338",
  "term_id": "GO:0004459",
  "term_label": "L-lactate dehydrogenase (NAD+) activity",
  "gene_name": "L-lactate dehydrogenase A chain",
  "gene_symbol": "LDHA"
}